PERK-mediated unfolded protein response [GO:0036499] (biological process) Also known as: PERK signal transduction pathway, PERK branch of UPR, PKR-like ER kinase signal transduction, UPR signaling by PERK stress sensor, endoplasmic reticulum unfolded protein response; PERK signaling, EIF2AK3-mediated unfolded protein response, PERK signaling in response to endoplasmic reticulum stress, eukaryotic translation initiation factor 2-alpha kinase 3-mediated unfolded protein response Relationships: is a type of ER-nucleus signaling pathway [GO:0006984]; is_a endoplasmic reticulum unfolded protein response [GO:0030968]; is a type of integrated stress response signaling [GO:0140467] Regulation: regulated by regulation of PERK-mediated unfolded protein response [GO:1903897]; negatively regulated by negative regulation of PERK-mediated unfolded protein response [GO:1903898]; positively regulated by positive regulation of PERK-mediated unfolded protein response [GO:1903899] References: PMID:22013210, PMID:27629041 Sources: GOC:PARL, GOC:bf Definition: The series of molecular signals mediated by the endoplasmic reticulum membrane stress sensor PERK (PKR-like ER kinase). Begins with activation of PERK in response to endoplasmic reticulum (ER) stress and ends with regulation of a downstream cellular process, e.g. transcription. The main substrate of PERK is the translation initiation factor eIF2alpha. Serine-phosphorylation of eIF2alpha by PERK inactivates eIF2alpha and inhibits general protein translation. In addition, eIF2alpha phosphorylation preferentially increases the translation of selective mRNAs such as ATF4 (activating transcription factor 4), which up regulates a subset of UPR genes required to restore folding capacity.